{
  "term_id": "GO:0072686",
  "gene": "UniProtKB:P52732",
  "gene_name": "Kinesin-like protein KIF11",
  "term_label": "mitotic spindle",
  "gene_symbol": "KIF11"
}